{
  "gene_name": "Sorbin and SH3 domain-containing protein 1",
  "term_label": "nucleus",
  "gene_symbol": "SORBS1",
  "gene": "UniProtKB:Q9BX66",
  "term_id": "GO:0005634"
}